{
  "gene_name": "5-hydroxytryptamine receptor 3D",
  "term_id": "GO:0005886",
  "gene": "UniProtKB:Q70Z44",
  "gene_symbol": "HTR3D",
  "term_label": "plasma membrane"
}